ladanein 6-O-methyltransferase activity [GO:0102535] (molecular function) Relationships: is a type of methyltransferase activity [GO:0008168] Definition: Catalysis of the reaction: ladanein + S-adenosyl-L-methionine = H+ + S-adenosyl-L-homocysteine + salvigenin. Sources: RHEA:73247